{
  "gene_name": "Dedicator of cytokinesis protein 5",
  "gene": "UniProtKB:Q9H7D0",
  "term_label": "cell migration",
  "gene_symbol": "DOCK5",
  "term_id": "GO:0016477"
}